{
  "term_label": "isopentenyl diphosphate biosynthetic process, mevalonate pathway",
  "gene": "UniProtKB:Q03426",
  "term_id": "GO:0019287",
  "gene_name": "Mevalonate kinase",
  "gene_symbol": "MVK"
}